{
  "gene_symbol": "FFAR3",
  "gene_name": "Free fatty acid receptor 3",
  "term_label": "G protein-coupled receptor activity",
  "gene": "UniProtKB:O14843",
  "term_id": "GO:0004930"
}